{
  "term_label": "detection of chemical stimulus involved in sensory perception of smell",
  "gene_name": "Olfactory receptor 2AJ1",
  "term_id": "GO:0050911",
  "gene_symbol": "OR2AJ1",
  "gene": "UniProtKB:Q8NGZ0"
}